{
  "gene": "UniProtKB:P21452",
  "gene_symbol": "TACR2",
  "term_label": "plasma membrane",
  "gene_name": "Substance-K receptor",
  "term_id": "GO:0005886"
}